{
  "term_id": "GO:0016712",
  "gene_symbol": "CYP2E1",
  "gene_name": "Cytochrome P450 2E1",
  "term_label": "oxidoreductase activity, acting on paired donors, with incorporation or reduction of molecular oxygen, reduced flavin or flavoprotein as one donor, and incorporation of one atom of oxygen",
  "gene": "UniProtKB:P05181"
}